{
  "term_id": "UNKNOWN:0001",
  "gene": "UniProtKB:Q86WS3",
  "term_label": "Unknown molecular function",
  "gene_symbol": "OOSP2",
  "gene_name": "Oocyte-secreted protein 2"
}